{
  "gene": "UniProtKB:Q9H9A6",
  "gene_name": "Leucine-rich repeat-containing protein 40",
  "gene_symbol": "LRRC40",
  "term_id": "UNKNOWN:0003",
  "term_label": "Unknown cellular component"
}